positive regulation of transcription from RNA polymerase II promoter by oleic acid [GO:0061429] (biological process) References: PMID:20395639 Sources: GOC:dph Definition: Any process involving oleic acid that activates or increases the frequency, rate or extent of transcription from an RNA polymerase II promoter. Relationships: is a type of carbon catabolite activation of transcription from RNA polymerase II promoter [GO:0000436]